{
  "gene_name": "Dynamin-like 120 kDa protein, mitochondrial",
  "gene": "UniProtKB:O60313",
  "gene_symbol": "OPA1",
  "term_label": "microtubule",
  "term_id": "GO:0005874"
}